{
  "gene_name": "Collagen alpha-2(VI) chain",
  "term_label": "Unknown molecular function",
  "term_id": "UNKNOWN:0001",
  "gene_symbol": "COL6A2",
  "gene": "UniProtKB:P12110"
}